{
  "gene": "UniProtKB:O14657",
  "gene_symbol": "TOR1B",
  "gene_name": "Torsin-1B",
  "term_label": "protein localization to nucleus",
  "term_id": "GO:0034504"
}